negative regulation of smoothened signaling pathway involved in dorsal/ventral neural tube patterning [GO:1901621] (biological process) Sources: GOC:TermGenie Also known as: down regulation of hedgehog signaling pathway involved in dorsal/ventral neural tube patterning, down regulation of hh signaling pathway involved in dorsal/ventral neural tube patterning, down regulation of smoothened signaling pathway involved in dorsal/ventral neural tube patterning, down regulation of smoothened signalling pathway involved in dorsal/ventral neural tube patterning, down-regulation of hedgehog signaling pathway involved in dorsal/ventral neural tube patterning, down-regulation of hh signaling pathway involved in dorsal/ventral neural tube patterning, down-regulation of smoothened signaling pathway involved in dorsal/ventral neural tube patterning, down-regulation of smoothened signalling pathway involved in dorsal/ventral neural tube patterning, downregulation of hedgehog signaling pathway involved in dorsal/ventral neural tube patterning, downregulation of hh signaling pathway involved in dorsal/ventral neural tube patterning, downregulation of smoothened signaling pathway involved in dorsal/ventral neural tube patterning, downregulation of smoothened signalling pathway involved in dorsal/ventral neural tube patterning, negative regulation of hedgehog signaling pathway involved in dorsal/ventral neural tube patterning, negative regulation of hh signaling pathway involved in dorsal/ventral neural tube patterning, negative regulation of smoothened signalling pathway involved in dorsal/ventral neural tube patterning, inhibition of hedgehog signaling pathway involved in dorsal/ventral neural tube patterning, inhibition of hh signaling pathway involved in dorsal/ventral neural tube patterning, inhibition of smoothened signaling pathway involved in dorsal/ventral neural tube patterning, inhibition of smoothened signalling pathway involved in dorsal/ventral neural tube patterning Definition: Any process that stops, prevents or reduces the frequency, rate or extent of smoothened signaling pathway involved in dorsal/ventral neural tube patterning. Relationships: is a type of GO:0045879; is a type of regulation of smoothened signaling pathway involved in dorsal/ventral neural tube patterning [GO:1901620]; negatively regulates smoothened signaling pathway involved in dorsal/ventral neural tube patterning [GO:0060831]